23S rRNA (guanine(745)-N(1))-methyltransferase activity [GO:0052911] (molecular function) Definition: Catalysis of the reaction: S-adenosyl-L-methionine + guanine(745) in 23S rRNA = N(1)-methylguanine(745) in 23S rRNA + S-adenosyl-L-homocysteine. Also known as: S-adenosyl-L-methionine:rRNA (guanine-1-N-)-methyltransferase activity, rRNA(m(1)G)methylase activity, ribosomal RNA(m(1)G)-methylase activity, ribosomal ribonucleate guanine 1-methyltransferase activity, rlmA(I) methyltransferase activity, 23S rRNA m(1)G(745) methyltransferase activity Sources: EC:2.1.1.187 Relationships: is a type of rRNA (guanine-N1-)-methyltransferase activity [GO:0008989]